phosphoenolpyruvate-dependent sugar phosphotransferase complex [GO:0019197] (cellular component) Definition: Includes phosphoenolpyruvate-protein phosphatase (enzyme I of the phosphotransferase system) and protein-N(PI)-phosphohistidine-sugar phosphotransferase (enzyme II of the phosphotransferase system). Sources: GOC:ma Relationships: is a type of GO:1902494; is part of cytoplasm [GO:0005737]